{
  "term_label": "basolateral plasma membrane",
  "gene_symbol": "SLC4A10",
  "gene_name": "Sodium-driven chloride bicarbonate exchanger",
  "gene": "UniProtKB:Q6U841",
  "term_id": "GO:0016323"
}